{
  "gene_symbol": "SFTPA2",
  "gene": "UniProtKB:Q8IWL1",
  "gene_name": "Pulmonary surfactant-associated protein A2",
  "term_label": "Unknown molecular function",
  "term_id": "UNKNOWN:0001"
}